{
  "term_label": "vascular endothelial growth factor receptor signaling pathway",
  "term_id": "GO:0048010",
  "gene": "UniProtKB:P49765",
  "gene_symbol": "VEGFB",
  "gene_name": "Vascular endothelial growth factor B"
}